{
  "gene": "UniProtKB:Q9NPJ6",
  "gene_name": "Mediator of RNA polymerase II transcription subunit 4",
  "term_label": "regulation of transcription by RNA polymerase II",
  "gene_symbol": "MED4",
  "term_id": "GO:0006357"
}